cis-stilbene-oxide hydrolase activity [GO:0033961] (molecular function) Relationships: is a type of epoxide hydrolase activity [GO:0004301] Definition: Catalysis of the reaction: cis-stilbene oxide + H2O = (+)-(1R,2R)-1,2-diphenylethane-1,2-diol. Also known as: arene-oxide hydratase activity, aryl epoxide hydrase activity, epoxide hydrase activity, epoxide hydratase activity, benzo(a)pyrene-4,5-epoxide hydratase activity, benzo[a]pyrene-4,5-oxide hydratase activity, microsomal epoxide hydrase activity, microsomal epoxide hydratase activity, microsomal epoxide hydrolase activity, cis-epoxide hydrolase activity, mEH Sources: EC:3.3.2.9